{
  "gene_name": "Extracellular calcium-sensing receptor",
  "gene_symbol": "CASR",
  "term_label": "plasma membrane",
  "gene": "UniProtKB:P41180",
  "term_id": "GO:0005886"
}